cytosolic proteasome regulatory particle, lid subcomplex [GO:0031615] (cellular component) Definition: The subcomplex of the cytosolic proteasome regulatory particle that forms the peripheral lid, which is added on top of the base subcomplex. Sources: GOC:mah, GOC:mtg_sensu Relationships: is a type of proteasome regulatory particle, lid subcomplex [GO:0008541]; is part of GO:0031600